{
  "term_label": "regulation of transcription by RNA polymerase II",
  "gene_name": "Zinc finger protein 524",
  "gene": "UniProtKB:Q96C55",
  "gene_symbol": "ZNF524",
  "term_id": "GO:0006357"
}